{
  "gene_name": "Mothers against decapentaplegic homolog 3",
  "gene": "UniProtKB:P84022",
  "term_label": "transforming growth factor beta receptor signaling pathway",
  "term_id": "GO:0007179",
  "gene_symbol": "SMAD3"
}